{
  "term_label": "poly(A)+ mRNA export from nucleus",
  "gene_symbol": "NXF5",
  "gene": "UniProtKB:Q9H1B4",
  "term_id": "GO:0016973",
  "gene_name": "Nuclear RNA export factor 5"
}